{
  "term_id": "GO:0007099",
  "gene_symbol": "RTTN",
  "gene": "UniProtKB:Q86VV8",
  "gene_name": "Rotatin",
  "term_label": "centriole replication"
}